phenylacetyl-CoA 1,2-epoxidase complex [GO:0062077] (cellular component) Also known as: paaABCE complex Relationships: is a type of oxidoreductase complex [GO:1990204] References: PMID:21247899 Sources: GOC:bhm Definition: A protein complex capable of catalysing the reaction: phenylacetyl-CoA + H+ + NADPH + O2 = 2-(1,2-epoxy-1,2-dihydrophenyl)acetyl-CoA + H2O + NADP+.